{
  "gene_name": "Mitochondrial import receptor subunit TOM70",
  "term_id": "GO:0030150",
  "gene": "UniProtKB:O94826",
  "term_label": "protein import into mitochondrial matrix",
  "gene_symbol": "TOMM70"
}